{
  "term_id": "GO:0031005",
  "gene": "UniProtKB:Q6ZTI6",
  "gene_name": "Refilin-A",
  "gene_symbol": "RFLNA",
  "term_label": "filamin binding"
}